{
  "gene_name": "Putative mitochondrial transporter UCP3",
  "term_id": "GO:1990542",
  "gene": "UniProtKB:P55916",
  "term_label": "mitochondrial transmembrane transport",
  "gene_symbol": "UCP3"
}